{
  "gene_symbol": "RMI2",
  "term_id": "GO:0005829",
  "gene_name": "RecQ-mediated genome instability protein 2",
  "term_label": "cytosol",
  "gene": "UniProtKB:Q96E14"
}